{
  "term_label": "Unknown biological process",
  "gene_symbol": "CDKN2D",
  "term_id": "UNKNOWN:0002",
  "gene_name": "Cyclin-dependent kinase 4 inhibitor D",
  "gene": "UniProtKB:P55273"
}